{
  "term_label": "serine-type endopeptidase activity",
  "gene": "UniProtKB:Q92876",
  "gene_name": "Kallikrein-6",
  "gene_symbol": "KLK6",
  "term_id": "GO:0004252"
}